{
  "term_id": "GO:0008104",
  "term_label": "intracellular protein localization",
  "gene_name": "Protein odr-4 homolog",
  "gene_symbol": "ODR4",
  "gene": "UniProtKB:Q5SWX8"
}